positive regulation of promoter clearance from RNA polymerase II promoter [GO:0140846] (biological process) References: PMID:28248323 Relationships: is a type of regulation of promoter clearance from RNA polymerase II promoter [GO:0140845]; is a type of positive regulation of RNA biosynthetic process [GO:1902680]; positively regulates GO:0001111 Definition: A process that activates or increases the frequency, rate or extent of the transition from the initiation to the elongation phases of transcription by RNA polymerase II.